{
  "gene_name": "Microtubule-associated serine_threonine-protein kinase 4",
  "term_label": "microtubule cytoskeleton",
  "term_id": "GO:0015630",
  "gene": "UniProtKB:O15021",
  "gene_symbol": "MAST4"
}